negative regulation of lactose biosynthetic process [GO:1903535] (biological process) Definition: Any process that stops, prevents or reduces the frequency, rate or extent of lactose biosynthetic process. Relationships: is a type of negative regulation of biosynthetic process [GO:0009890]; is a type of negative regulation of carbohydrate metabolic process [GO:0045912]; is a type of regulation of lactose biosynthetic process [GO:1903534]; negatively regulates lactose biosynthetic process [GO:0005989] Also known as: down regulation of lactose anabolism, down regulation of lactose biosynthesis, down regulation of lactose biosynthetic process, down regulation of lactose formation, down regulation of lactose synthesis, down-regulation of lactose anabolism, down-regulation of lactose biosynthesis, down-regulation of lactose biosynthetic process, down-regulation of lactose formation, down-regulation of lactose synthesis, downregulation of lactose anabolism, downregulation of lactose biosynthesis, downregulation of lactose biosynthetic process, downregulation of lactose formation, downregulation of lactose synthesis, negative regulation of lactose anabolism, negative regulation of lactose biosynthesis, negative regulation of lactose formation, negative regulation of lactose synthesis, inhibition of lactose anabolism, inhibition of lactose biosynthesis, inhibition of lactose biosynthetic process, inhibition of lactose formation, inhibition of lactose synthesis References: PMID:12018418 Sources: GOC:TermGenie, GOC:mr, GO_REF:0000058